{
  "term_id": "GO:0005886",
  "gene_symbol": "PI4K2B",
  "gene_name": "Phosphatidylinositol 4-kinase type 2-beta",
  "term_label": "plasma membrane",
  "gene": "UniProtKB:Q8TCG2"
}